bicoid mRNA localization [GO:0045450] (biological process) Definition: Any process in which bicoid mRNA is transported to and maintained within the oocyte as part of the specification of the anterior/posterior axis. Regulation: regulated by regulation of bicoid mRNA localization [GO:0008359]; negatively regulated by negative regulation of bicoid mRNA localization [GO:0045853]; RO_0002213 by positive regulation of bicoid mRNA localization [GO:0045854] Also known as: bicoid mRNA localisation, establishment and maintenance of bicoid mRNA localization Relationships: is a type of intracellular mRNA localization involved in anterior/posterior axis specification [GO:0060811]; is part of GO:0007314 Sources: GOC:go_curators